trigeminal ganglion formation [GO:0061561] (biological process) Relationships: is a type of cranial ganglion formation [GO:0061560]; is part of trigeminal ganglion morphogenesis [GO:0061556] Also known as: trigeminal ganglia formation Definition: The process that gives rise to the trigeminal ganglion. This process pertains to the initial formation of a structure from unspecified parts. Sources: GOC:dph